ribonucleoside diphosphate metabolic process [GO:0009185] (biological process) Subtypes: purine ribonucleoside diphosphate metabolic process [GO:0009179], ribonucleoside diphosphate biosynthetic process [GO:0009188], GO:0009191, pyrimidine ribonucleoside diphosphate metabolic process [GO:0009193] Also known as: ribonucleoside diphosphate metabolism Definition: The chemical reactions and pathways involving a ribonucleoside diphosphate, a compound consisting of a nucleobase linked to a ribose sugar esterified with diphosphate on the sugar. Sources: GOC:go_curators, ISBN:0198506732 Relationships: is a type of GO:0009132